regulation of vasculogenesis [GO:2001212] (biological process) Definition: Any process that modulates the frequency, rate or extent of vasculogenesis. Subtypes: negative regulation of vasculogenesis [GO:2001213], GO:2001214 Also known as: regulation of vascular morphogenesis Relationships: is a type of regulation of cell differentiation [GO:0045595]; regulates GO:0001570 Sources: GOC:obol